{
  "gene": "UniProtKB:Q8NH89",
  "gene_name": "Putative olfactory receptor 5AK3",
  "term_id": "UNKNOWN:0003",
  "gene_symbol": "OR5AK3P",
  "term_label": "Unknown cellular component"
}